{
  "gene_symbol": "CALHM2",
  "gene_name": "Calcium homeostasis modulator protein 2",
  "term_label": "Unknown biological process",
  "term_id": "UNKNOWN:0002",
  "gene": "UniProtKB:Q9HA72"
}